{
  "term_label": "semaphorin-plexin signaling pathway",
  "gene": "UniProtKB:O60486",
  "gene_name": "Plexin-C1",
  "term_id": "GO:0071526",
  "gene_symbol": "PLXNC1"
}